{
  "gene_name": "Potassium voltage-gated channel subfamily G member 4",
  "term_label": "voltage-gated potassium channel complex",
  "gene_symbol": "KCNG4",
  "gene": "UniProtKB:Q8TDN1",
  "term_id": "GO:0008076"
}